{
  "term_id": "GO:0006511",
  "gene_symbol": "RNF5",
  "gene": "UniProtKB:Q99942",
  "term_label": "ubiquitin-dependent protein catabolic process",
  "gene_name": "E3 ubiquitin-protein ligase RNF5"
}